{
  "gene_name": "Calcyphosin-like protein",
  "gene": "UniProtKB:Q8WWF8",
  "term_id": "UNKNOWN:0001",
  "term_label": "Unknown molecular function",
  "gene_symbol": "CAPSL"
}